{
  "term_id": "UNKNOWN:0003",
  "gene": "UniProtKB:Q5GAN4",
  "gene_symbol": "RNASE12",
  "term_label": "Unknown cellular component",
  "gene_name": "Probable inactive ribonuclease-like protein 12"
}